negative regulation of oospore formation [GO:0075246] (biological process) Relationships: is a type of negative regulation of sexual sporulation resulting in formation of a cellular spore [GO:0043942]; is a type of regulation of oospore formation [GO:0075244]; negatively regulates oospore formation [GO:0075243] Sources: GOC:pamgo_curators Definition: Any process that stops, prevents, or reduces the frequency, rate or extent of oospore formation, a process in which male and female gametangia develop and fuse to form a thick-walled resting spore of oomycetes.